detection of reduced oxygen by aortic body chemoreceptor signaling [GO:0003038] (biological process) Sources: GOC:mtg_cardio Definition: The process in which information about the levels of oxygen are received and are converted to a molecular signal by chemoreceptors in an aortic body. Also known as: detection of reduced oxygen by aortic body chemoreceptor signalling Relationships: is a type of GO:0003020; is part of detection of hypoxic conditions in blood by aortic body chemoreceptor signaling [GO:0003033]